{
  "gene": "UniProtKB:P30281",
  "term_label": "G1/S transition of mitotic cell cycle",
  "term_id": "GO:0000082",
  "gene_symbol": "CCND3",
  "gene_name": "G1_S-specific cyclin-D3"
}